{
  "term_id": "GO:0035556",
  "term_label": "intracellular signal transduction",
  "gene_name": "Serine_threonine-protein kinase WNK3",
  "gene": "UniProtKB:Q9BYP7",
  "gene_symbol": "WNK3"
}